{
  "gene_symbol": "WWTR1",
  "term_id": "GO:0003713",
  "term_label": "transcription coactivator activity",
  "gene": "UniProtKB:Q9GZV5",
  "gene_name": "WW domain-containing transcription regulator protein 1"
}